response to serotonin [GO:1904014] (biological process) References: PMID:1505525 Sources: GOC:TermGenie, GO_REF:0000071 Subtypes: cellular response to serotonin [GO:1904015] Definition: Any process that results in a change in state or activity of a cell or an organism (in terms of movement, secretion, enzyme production, gene expression, etc.) as a result of a serotonin stimulus. Relationships: is a type of response to monoamine [GO:0071867]; is a type of response to oxygen-containing compound [GO:1901700]